{
  "gene": "UniProtKB:P47869",
  "term_label": "gamma-aminobutyric acid signaling pathway",
  "gene_name": "Gamma-aminobutyric acid receptor subunit alpha-2",
  "gene_symbol": "GABRA2",
  "term_id": "GO:0007214"
}